regulation of tissue remodeling [GO:0034103] (biological process) Subtypes: GO:0034104, GO:0034105, regulation of erythrocyte clearance [GO:0034106], regulation of bone remodeling [GO:0046850], regulation of blood vessel remodeling [GO:0060312], regulation of mammary gland involution [GO:1903519], regulation of connective tissue replacement [GO:1905203] Relationships: is a type of regulation of multicellular organismal process [GO:0051239]; regulates GO:0048771 Sources: GOC:add Also known as: regulation of tissue remodelling Definition: Any process that modulates the frequency, rate, or extent of tissue remodeling.